{
  "gene_name": "Autophagy-related protein 2 homolog A",
  "term_id": "GO:0000045",
  "gene_symbol": "ATG2A",
  "term_label": "autophagosome assembly",
  "gene": "UniProtKB:Q2TAZ0"
}